ergosterol biosynthetic process [GO:0006696] (BP) Sources: ISBN:0198506732 Regulation: negatively regulated by negative regulation of ergosterol biosynthetic process [GO:0010895]; regulated by regulation of ergosterol biosynthetic process [GO:0032443]; positively regulated by positive regulation of ergosterol biosynthetic process [GO:0070452] Relationships: is a type of GO:0008204; is a type of sterol biosynthetic process [GO:0016126]; is a type of GO:0016129; is a type of secondary alcohol biosynthetic process [GO:1902653] Also known as: ergosterol anabolism, ergosterol biosynthesis, ergosterol formation, ergosterol synthesis Definition: The chemical reactions and pathways resulting in the formation of ergosterol, (22E)-ergosta-5,7,22-trien-3-beta-ol, a sterol found in ergot, yeast and moulds.